venom-mediated myocyte killing in another organism [GO:0044522] (biological process) Definition: A process that begins with venom being forced into an organism by the bite or sting of another organism, killing heart myocytes and ultimately resulting in muscle damage in the bitten organism. Relationships: is_a GO:0031640; is a type of GO:0044521 References: PMID:10620318, PMID:21150580 Sources: GOC:fj, GOC:jl Also known as: envenomation resulting in myocyte killing causing muscle damage in other organism, envenomation resulting in myocyte killing in another organism, envenomation resulting in myocyte killing in other organism